{
  "gene": "UniProtKB:O94953",
  "term_id": "GO:0010468",
  "term_label": "regulation of gene expression",
  "gene_symbol": "KDM4B",
  "gene_name": "Lysine-specific demethylase 4B"
}